{
  "term_id": "GO:2000369",
  "gene_name": "AP2-associated protein kinase 1",
  "gene": "UniProtKB:Q2M2I8",
  "gene_symbol": "AAK1",
  "term_label": "regulation of clathrin-dependent endocytosis"
}